{
  "gene_name": "Epidermal growth factor receptor substrate 15-like 1",
  "gene": "UniProtKB:Q9UBC2",
  "gene_symbol": "EPS15L1",
  "term_label": "endocytosis",
  "term_id": "GO:0006897"
}